{
  "gene_symbol": "C4orf17",
  "gene": "UniProtKB:Q53FE4",
  "gene_name": "Uncharacterized protein C4orf17",
  "term_label": "Unknown cellular component",
  "term_id": "UNKNOWN:0003"
}